wing disc dorsal/ventral pattern formation [GO:0048190] (biological process) Also known as: wing disc dorsal-ventral pattern formation, wing disc dorsoventral pattern formation Sources: GOC:jid Relationships: is a type of GO:0007450; is_a wing disc pattern formation [GO:0035222] Definition: The establishment, maintenance and elaboration of the dorsal/ventral axis of the wing disc, a precursor to the adult wing.